response to water deprivation [GO:0009414] (BP) Sources: GOC:lr Subtypes: response to desiccation [GO:0009269], drought recovery [GO:0009819], cellular response to water deprivation [GO:0042631] Also known as: response to dehydration, response to drought, response to thirst, drought tolerance Relationships: is_a response to stress [GO:0006950]; is a type of response to water [GO:0009415] Regulation: negatively regulated by GO:0080148; positively regulated by GO:1902584; regulated by regulation of response to water deprivation [GO:2000070] Definition: Any process that results in a change in state or activity of a cell or an organism (in terms of movement, secretion, enzyme production, gene expression, etc.) as a result of a water deprivation stimulus, prolonged deprivation of water.